{
  "gene": "UniProtKB:Q8ND56",
  "term_id": "GO:0033962",
  "term_label": "P-body assembly",
  "gene_name": "Protein LSM14 homolog A",
  "gene_symbol": "LSM14A"
}